{
  "gene_symbol": "TBC1D5",
  "term_id": "GO:0005794",
  "term_label": "Golgi apparatus",
  "gene": "UniProtKB:Q92609",
  "gene_name": "TBC1 domain family member 5"
}